{
  "gene_symbol": "MORN1",
  "term_label": "Unknown biological process",
  "term_id": "UNKNOWN:0002",
  "gene_name": "MORN repeat-containing protein 1",
  "gene": "UniProtKB:Q5T089"
}